{
  "term_id": "GO:0008076",
  "gene": "UniProtKB:Q8TDN2",
  "gene_symbol": "KCNV2",
  "term_label": "voltage-gated potassium channel complex",
  "gene_name": "Potassium voltage-gated channel subfamily V member 2"
}